biotin binding [GO:0009374] (molecular function) Definition: Binding to biotin (cis-tetrahydro-2-oxothieno(3,4-d)imidazoline-4-valeric acid), the (+) enantiomer of which is very widely distributed in cells and serves as a carrier in a number of enzymatic beta-carboxylation reactions. Relationships: is_a GO:0019842; is a type of amide binding [GO:0033218]; is a type of monocarboxylic acid binding [GO:0033293]; is a type of GO:1901363; is a type of GO:1901681 Also known as: vitamin B7 binding, vitamin H binding Sources: GOC:jl, ISBN:0198506732